accessory outer segment [GO:1990906] (cellular component) Relationships: is a type of neuron projection [GO:0043005] References: PMID:25125189 Sources: GOC:dph Definition: A cilium-like cell projection emanating from the inner segment and running alongside the outer segment of photoreceptors.